{
  "gene_symbol": "NCAPD3",
  "term_id": "GO:0000779",
  "term_label": "condensed chromosome, centromeric region",
  "gene_name": "Condensin-2 complex subunit D3",
  "gene": "UniProtKB:P42695"
}